{
  "term_id": "GO:0005759",
  "gene_name": "Nardilysin",
  "gene": "UniProtKB:O43847",
  "gene_symbol": "NRDC",
  "term_label": "mitochondrial matrix"
}